regulation of receptor localization to synapse [GO:1902683] (biological process) Definition: Any process that modulates the frequency, rate or extent of receptor localization to synapse. References: PMID:22252129 Sources: GOC:TermGenie, GOC:kmv, GO_REF:0000058 Also known as: regulation of receptor localisation to synapse Relationships: is a type of regulation of localization [GO:0032879]; regulates receptor localization to synapse [GO:0097120] Subtypes: regulation of neurotransmitter receptor localization to postsynaptic specialization membrane [GO:0098696], regulation of exocytic insertion of neurotransmitter receptor to postsynaptic membrane [GO:0099145], regulation of neurotransmitter receptor transport, endosome to postsynaptic membrane [GO:0099152], regulation of postsynaptic neurotransmitter receptor diffusion trapping [GO:0150054], negative regulation of receptor localization to synapse [GO:1902684], GO:1902685